{
  "gene_name": "Uncharacterized protein KIAA2013",
  "gene_symbol": "KIAA2013",
  "term_label": "Unknown biological process",
  "gene": "UniProtKB:Q8IYS2",
  "term_id": "UNKNOWN:0002"
}